{
  "gene_name": "Nidogen-2",
  "gene_symbol": "NID2",
  "term_label": "Unknown molecular function",
  "term_id": "UNKNOWN:0001",
  "gene": "UniProtKB:Q14112"
}